{
  "term_label": "long-chain fatty acid import into peroxisome",
  "gene": "UniProtKB:P33897",
  "term_id": "GO:0015910",
  "gene_symbol": "ABCD1",
  "gene_name": "ATP-binding cassette sub-family D member 1"
}